{
  "gene_symbol": "VCAN",
  "gene": "UniProtKB:P13611",
  "term_label": "synapse",
  "term_id": "GO:0045202",
  "gene_name": "Versican core protein"
}